{
  "gene_symbol": "PRKAA1",
  "term_label": "cellular response to glucose starvation",
  "term_id": "GO:0042149",
  "gene_name": "5'-AMP-activated protein kinase catalytic subunit alpha-1",
  "gene": "UniProtKB:Q13131"
}